alphaIIb-beta3 integrin-CD47-FAK complex [GO:0070770] (cellular component) Relationships: is a type of plasma membrane protein complex [GO:0098797] References: PMID:9169439 Also known as: ITGA2b-ITGB3-CD47-FAK complex Definition: A protein complex that consists of an alphaIIb-beta3 integrin complex bound to the cell surface antigen CD47 and the kinase FAK.